{
  "gene_name": "Single-pass membrane and coiled-coil domain-containing protein 1",
  "term_label": "Unknown molecular function",
  "gene_symbol": "SMCO1",
  "gene": "UniProtKB:Q147U7",
  "term_id": "UNKNOWN:0001"
}